positive regulation of synaptic vesicle uncoating [GO:1903390] (biological process) Definition: Any process that activates or increases the frequency, rate or extent of synaptic vesicle uncoating. Relationships: is a type of positive regulation of protein depolymerization [GO:1901881]; is a type of regulation of synaptic vesicle uncoating [GO:1903388]; positively regulates synaptic vesicle uncoating [GO:0016191] References: PMID:21563316 Sources: GOC:PARL, GOC:TermGenie, GOC:pad, GO_REF:0000058 Also known as: positive regulation of synaptic vesicle coat depolymerization, positive regulation of synaptic vesicle coat protein depolymerization, up regulation of synaptic vesicle coat depolymerization, up regulation of synaptic vesicle coat protein depolymerization, up regulation of synaptic vesicle uncoating, up-regulation of synaptic vesicle coat depolymerization, up-regulation of synaptic vesicle coat protein depolymerization, up-regulation of synaptic vesicle uncoating, upregulation of synaptic vesicle coat depolymerization, upregulation of synaptic vesicle coat protein depolymerization, upregulation of synaptic vesicle uncoating, activation of synaptic vesicle coat depolymerization, activation of synaptic vesicle coat protein depolymerization, activation of synaptic vesicle uncoating